intermembrane lipid transfer [GO:0120009] (biological process) Definition: The transport of lipids between membranes in which a lipid molecule is transported through an aqueous phase from the outer leaflet of a donor membrane to the outer leaflet of an acceptor membrane. This process does not require metabolic energy and can be either spontaneous or mediated by lipid transfer proteins (LTPs). References: PMID:20823909, PMID:24220498, PMID:25797198 Sources: GOC:krc Relationships: is a type of lipid transport [GO:0006869]; is a type of GO:0061024 Subtypes: intermembrane phospholipid transfer [GO:0120010], GO:0120011, intermembrane sphingolipid transfer [GO:0120012]